{
  "gene_symbol": "ATP8B1",
  "term_id": "GO:0045332",
  "term_label": "phospholipid translocation",
  "gene": "UniProtKB:O43520",
  "gene_name": "Phospholipid-transporting ATPase IC"
}